DNA replication preinitiation complex assembly [GO:0071163] (biological process) Definition: The aggregation, arrangement and bonding together of a set of components to form the DNA replication preinitiation complex, a protein-DNA complex that is assembled at DNA replication origins as part of initiation of DNA replication. The complex consists of proteins that initiate the DNA binding, melt the helix and enable helicase activity. Subtypes: GO:0071165, CMG complex assembly [GO:0140529], premeiotic DNA replication preinitiation complex assembly [GO:1902976], mitotic DNA replication preinitiation complex assembly [GO:1902977] References: PMID:28209641 Sources: GOC:mah Relationships: is a type of GO:0022402; is a type of protein-DNA complex assembly [GO:0065004]; is part of nuclear DNA replication [GO:0033260] Also known as: DNA replication preinitiation complex formation, pre-IC complex assembly